{
  "gene_name": "Olfactory receptor 13C8",
  "term_label": "detection of chemical stimulus involved in sensory perception of smell",
  "gene": "UniProtKB:Q8NGS7",
  "gene_symbol": "OR13C8",
  "term_id": "GO:0050911"
}